{
  "gene_name": "Unconventional myosin-XV",
  "gene_symbol": "MYO15A",
  "gene": "UniProtKB:Q9UKN7",
  "term_id": "GO:0098858",
  "term_label": "actin-based cell projection"
}